{
  "term_id": "GO:0007200",
  "gene": "UniProtKB:P34981",
  "gene_name": "Thyrotropin-releasing hormone receptor",
  "term_label": "phospholipase C-activating G protein-coupled receptor signaling pathway",
  "gene_symbol": "TRHR"
}